{
  "gene": "UniProtKB:O43805",
  "gene_symbol": "SSNA1",
  "term_label": "axon extension",
  "gene_name": "Microtubule nucleation factor SSNA1",
  "term_id": "GO:0048675"
}